{
  "term_label": "nucleus",
  "gene_name": "Zinc finger protein GLIS1",
  "gene_symbol": "GLIS1",
  "gene": "UniProtKB:Q8NBF1",
  "term_id": "GO:0005634"
}